{
  "gene": "UniProtKB:Q13241",
  "gene_symbol": "KLRD1",
  "gene_name": "Natural killer cells antigen CD94",
  "term_label": "cell surface",
  "term_id": "GO:0009986"
}